{
  "term_id": "GO:0006357",
  "gene_name": "Estrogen receptor",
  "gene": "UniProtKB:P03372",
  "term_label": "regulation of transcription by RNA polymerase II",
  "gene_symbol": "ESR1"
}